{
  "term_label": "basolateral plasma membrane",
  "gene_symbol": "SLCO1B7",
  "gene_name": "Putative solute carrier organic anion transporter family member 1B7",
  "term_id": "GO:0016323",
  "gene": "UniProtKB:G3V0H7"
}